{
  "term_label": "peptide hormone processing",
  "gene_name": "Proprotein convertase subtilisin_kexin type 5",
  "gene": "UniProtKB:Q92824",
  "term_id": "GO:0016486",
  "gene_symbol": "PCSK5"
}